{
  "gene": "UniProtKB:P0CJ78",
  "term_label": "Unknown cellular component",
  "gene_symbol": "ZNF865",
  "gene_name": "Zinc finger protein 865",
  "term_id": "UNKNOWN:0003"
}